regulation of platelet-derived growth factor production [GO:0090361] (biological process) Sources: GOC:BHF Subtypes: positive regulation of platelet-derived growth factor production [GO:0090362] Definition: Any process that modulates the rate, frequency, or extent of the appearance of any platelet-derived growth factor due to biosynthesis or secretion following a cellular stimulus, resulting in an increase in its intracellular or extracellular levels. Relationships: is a type of regulation of cytokine production [GO:0001817]; regulates platelet-derived growth factor production [GO:0090360]